{
  "term_id": "GO:0016303",
  "term_label": "1-phosphatidylinositol-3-kinase activity",
  "gene_name": "Phosphatidylinositol 3-kinase C2 domain-containing subunit gamma",
  "gene": "UniProtKB:O75747",
  "gene_symbol": "PIK3C2G"
}